{
  "gene": "UniProtKB:Q9UBP8",
  "gene_symbol": "KAAG1",
  "term_id": "UNKNOWN:0003",
  "gene_name": "Kidney-associated antigen 1",
  "term_label": "Unknown cellular component"
}